response to abiotic stimulus [GO:0009628] (biological process) Subtypes: GO:0006970, response to temperature stimulus [GO:0009266], response to pH [GO:0009268], response to radiation [GO:0009314], GO:0009415, detection of abiotic stimulus [GO:0009582], response to mechanical stimulus [GO:0009612], response to gravity [GO:0009629], response to electrical stimulus [GO:0051602], response to oxygen levels [GO:0070482], response to magnetism [GO:0071000], cellular response to abiotic stimulus [GO:0071214], response to karrikin [GO:0080167], invasive growth in response to abiotic stimulus [GO:0097318], response to viscosity [GO:0097714] Sources: GOC:hb Relationships: is a type of response to stimulus [GO:0050896] Also known as: response to abiotic stress Definition: Any process that results in a change in state or activity of a cell or an organism (in terms of movement, secretion, enzyme production, gene expression, etc.) as a result of an abiotic (not derived from living organisms) stimulus. Note: Note that this term is in the subset of terms that should not be used for direct gene product annotation. Instead, select a child term or, if no appropriate child term exists, please request a new term. Direct annotations to this term may be amended during annotation QC.